{
  "gene_symbol": "LZTFL1",
  "term_id": "GO:0030317",
  "term_label": "flagellated sperm motility",
  "gene": "UniProtKB:Q9NQ48",
  "gene_name": "Leucine zipper transcription factor-like protein 1"
}